{
  "gene_symbol": "PAIP1",
  "term_label": "regulation of translational initiation",
  "gene_name": "Polyadenylate-binding protein-interacting protein 1",
  "term_id": "GO:0006446",
  "gene": "UniProtKB:Q9H074"
}